{
  "gene_name": "Growth hormone-regulated TBC protein 1",
  "gene": "UniProtKB:Q5TC63",
  "term_id": "GO:0005096",
  "gene_symbol": "GRTP1",
  "term_label": "GTPase activator activity"
}